{
  "gene_name": "Single-stranded DNA cytosine deaminase",
  "term_label": "RNA binding",
  "gene_symbol": "AICDA",
  "term_id": "GO:0003723",
  "gene": "UniProtKB:Q9GZX7"
}